{
  "gene_name": "Protein ERGIC-53-like",
  "term_label": "COPII-coated ER to Golgi transport vesicle",
  "gene": "UniProtKB:Q9HAT1",
  "gene_symbol": "LMAN1L",
  "term_id": "GO:0030134"
}